metanephric proximal straight tubule development [GO:0072230] (biological process) Definition: The process whose specific outcome is the progression of the metanephric proximal straight tubule over time, from its formation to the mature structure. The metanephric proximal straight tubule is the part of the metanephric descending limb that extends from the metanephric proximal convoluted tubule to the metanephric descending thin tubule. Also known as: metanephric S3 development Sources: GOC:mtg_kidney_jan10 Relationships: is a type of proximal straight tubule development [GO:0072020]; is a type of GO:0072234; is part of GO:0072237